{
  "gene_name": "Monocarboxylate transporter 3",
  "term_id": "GO:0008028",
  "gene": "UniProtKB:O95907",
  "gene_symbol": "SLC16A8",
  "term_label": "monocarboxylic acid transmembrane transporter activity"
}